{
  "gene": "UniProtKB:Q7Z7N9",
  "gene_symbol": "TMEM179B",
  "gene_name": "Transmembrane protein 179B",
  "term_label": "Unknown cellular component",
  "term_id": "UNKNOWN:0003"
}